{
  "term_id": "GO:0004879",
  "gene_name": "Retinoic acid receptor gamma",
  "gene": "UniProtKB:P13631",
  "gene_symbol": "RARG",
  "term_label": "nuclear receptor activity"
}